{
  "gene_symbol": "LPCAT1",
  "gene_name": "Lysophosphatidylcholine acyltransferase 1",
  "term_label": "Unknown biological process",
  "term_id": "UNKNOWN:0002",
  "gene": "UniProtKB:Q8NF37"
}